{
  "term_label": "cytoplasm",
  "gene_name": "Kelch-like protein 21",
  "gene": "UniProtKB:Q9UJP4",
  "term_id": "GO:0005737",
  "gene_symbol": "KLHL21"
}